{
  "term_label": "transmembrane signaling receptor activity",
  "gene_name": "B-cell antigen receptor complex-associated protein alpha chain",
  "term_id": "GO:0004888",
  "gene": "UniProtKB:P11912",
  "gene_symbol": "CD79A"
}